{
  "term_id": "GO:0003712",
  "gene": "UniProtKB:D6RGH6",
  "gene_name": "Multicilin",
  "term_label": "transcription coregulator activity",
  "gene_symbol": "MCIDAS"
}